{
  "gene_symbol": "NUFIP2",
  "term_id": "UNKNOWN:0002",
  "term_label": "Unknown biological process",
  "gene": "UniProtKB:Q7Z417",
  "gene_name": "FMR1-interacting protein NUFIP2"
}